Atg12-Atg5-Atg16 complex [GO:0034274] (cellular component) References: PMID:17986448 Sources: GOC:rb Definition: A protein complex required for the expansion of the autophagosomal membrane. In budding yeast, this complex consists of Atg12p, Atg5p and Atg16p. Relationships: is a type of transferase complex [GO:1990234]; is part of cytoplasm [GO:0005737]